N6-acetyl-beta-lysine transaminase activity [GO:0047317] (molecular function) Sources: EC:2.6.1.65, MetaCyc:2.6.1.65-RXN Relationships: is a type of GO:0008483 Definition: Catalysis of the reaction: 2-oxoglutarate + 3-amino-6-acetamidohexanoate = L-glutamate + 3-oxo-6-acetamidohexanoate. Also known as: N6-acetyl-beta-lysine aminotransferase activity, 6-acetamido-3-aminohexanoate:2-oxoglutarate aminotransferase activity, N(6)-acetyl-beta-lysine aminotransferase activity, epsilon-acetyl-beta-lysine aminotransferase activity